{
  "term_id": "GO:0001228",
  "term_label": "DNA-binding transcription activator activity, RNA polymerase II-specific",
  "gene_name": "Forkhead box protein H1",
  "gene_symbol": "FOXH1",
  "gene": "UniProtKB:O75593"
}